{
  "gene_symbol": "MET",
  "term_label": "basal plasma membrane",
  "gene_name": "Hepatocyte growth factor receptor",
  "gene": "UniProtKB:P08581",
  "term_id": "GO:0009925"
}